{
  "term_label": "Unknown biological process",
  "gene": "UniProtKB:P49207",
  "term_id": "UNKNOWN:0002",
  "gene_name": "Large ribosomal subunit protein eL34",
  "gene_symbol": "RPL34"
}